{
  "gene_symbol": "PDGFA",
  "gene_name": "Platelet-derived growth factor subunit A",
  "term_label": "positive regulation of cell population proliferation",
  "gene": "UniProtKB:P04085",
  "term_id": "GO:0008284"
}